{
  "term_label": "benzodiazepine receptor activity",
  "gene": "UniProtKB:P18507",
  "gene_name": "Gamma-aminobutyric acid receptor subunit gamma-2",
  "term_id": "GO:0008503",
  "gene_symbol": "GABRG2"
}